ecdysone receptor holocomplex [GO:0008230] (cellular component) References: PMID:14592980 Sources: GOC:bf Definition: A heterodimeric complex containing the products of the insect genes Ecdysone receptor (EcR) and ultraspiracle (usp). Binding of ecdysone promotes association between the two subunits, and the receptor complex then initiates molting and metamorphosis by binding DNA and regulating the transcription of target genes. Relationships: is a type of RNA polymerase II transcription regulator complex [GO:0090575] Subtypes: repressor ecdysone receptor complex [GO:0008231], GO:0008232